antimonite transmembrane transporter activity [GO:0015104] (molecular function) Sources: GOC:ai Definition: Enables the transfer of antimonite from one side of a membrane to the other. Subtypes: antimonite secondary active transmembrane transporter activity [GO:0042960], ATPase-coupled antimonite transmembrane transporter activity [GO:0042961] Relationships: is a type of transmembrane transporter activity [GO:0022857]; is part of antimonite transmembrane transport [GO:0015699]